{
  "term_id": "GO:0060307",
  "gene_symbol": "KCNH2",
  "gene": "UniProtKB:Q12809",
  "term_label": "regulation of ventricular cardiac muscle cell membrane repolarization",
  "gene_name": "Potassium voltage-gated channel subfamily H member 2"
}